ornithine transmembrane import into vacuole [GO:0090455] (biological process) Sources: GOC:tb Definition: The directed movement of ornithine into the vacuole across the vacuolar membrane. Relationships: is a type of amino acid transmembrane transport [GO:0003333]; is a type of ornithine transport [GO:0015822]; is a type of vacuolar transmembrane transport [GO:0034486]; is a type of carboxylic acid transmembrane transport [GO:1905039] Also known as: vacuolar ornithine import